{
  "term_id": "GO:0034472",
  "term_label": "snRNA 3'-end processing",
  "gene_symbol": "SAGE2P",
  "gene_name": "Putative SAGE1-like protein",
  "gene": "UniProtKB:A6NJ88"
}